{
  "gene_name": "Calmodulin-2",
  "gene": "UniProtKB:P0DP24",
  "term_label": "centrosome",
  "term_id": "GO:0005813",
  "gene_symbol": "CALM2"
}